cellulosome binding [GO:1990300] (molecular function) Relationships: is a type of binding [GO:0005488] Also known as: scaffoldin complex binding Definition: Binding to a cellulosome, an extracellular multi-enzyme complex containing several enzymes aligned on a non-catalytic scaffolding that functions to hydrolyze plant cell wall polysaccharides. References: PMID:11893054, PMID:15197390 Sources: GOC:mengo_curators